{
  "gene_symbol": "COMMD8",
  "gene": "UniProtKB:Q9NX08",
  "gene_name": "COMM domain-containing protein 8",
  "term_id": "GO:0007165",
  "term_label": "signal transduction"
}